protein localization to synapse [GO:0035418] (biological process) Relationships: is a type of protein localization to cell junction [GO:1902414] Regulation: RO_0002211 by GO:1902473; RO_0002213 by positive regulation of protein localization to synapse [GO:1902474] Sources: GOC:bf Also known as: protein localisation to synapse Subtypes: protein localization to postsynapse [GO:0062237], gephyrin clustering involved in postsynaptic density assembly [GO:0097116], protein localization to presynapse [GO:1905383] Definition: Any process in which a protein is transported to, and/or maintained at the synapse, the junction between a nerve fiber of one neuron and another neuron or muscle fiber or glial cell.